{
  "gene_name": "CMP-N-acetylneuraminate-beta-galactosamide-alpha-2,3-sialyltransferase 1",
  "gene_symbol": "ST3GAL1",
  "term_label": "membrane",
  "gene": "UniProtKB:Q11201",
  "term_id": "GO:0016020"
}